lactose biosynthetic process [GO:0005989] (biological process) Relationships: is a type of lactose metabolic process [GO:0005988]; is a type of disaccharide biosynthetic process [GO:0046351] Also known as: lactose anabolism, lactose biosynthesis, lactose formation, lactose synthesis Sources: GOC:go_curators Definition: The chemical reactions and pathways resulting in the formation of lactose, the disaccharide galactopyranosyl-glucose. Regulation: regulated by regulation of lactose biosynthetic process [GO:1903534]; negatively regulated by negative regulation of lactose biosynthetic process [GO:1903535]; positively regulated by positive regulation of lactose biosynthetic process [GO:1903536]